diaminopimelate dehydrogenase activity [GO:0047850] (molecular function) Relationships: is a type of GO:0016639 Sources: EC:1.4.1.16, RHEA:13561 Definition: Catalysis of the reaction: meso-2,6-diaminopimelate + H2O + NADP+ = L-2-amino-6-oxopimelate + H+ + NADPH + NH4. Also known as: meso-2,6-diaminoheptanedioate:NADP+ oxidoreductase (deaminating), meso-alpha,epsilon-diaminopimelate dehydrogenase activity, meso-diaminopimelate D-dehydrogenase activity, meso-diaminopimelate dehydrogenase activity